{
  "gene_name": "LHFPL tetraspan subfamily member 7 protein",
  "term_label": "membrane",
  "gene_symbol": "LHFPL7",
  "term_id": "GO:0016020",
  "gene": "UniProtKB:Q6ICI0"
}